{
  "gene_symbol": "NWD1",
  "term_id": "UNKNOWN:0001",
  "gene": "UniProtKB:Q149M9",
  "term_label": "Unknown molecular function",
  "gene_name": "NACHT domain- and WD repeat-containing protein 1"
}